{
  "gene_name": "Eukaryotic translation initiation factor 3 subunit C-like protein",
  "gene_symbol": "EIF3CL",
  "term_id": "GO:0005852",
  "gene": "UniProtKB:B5ME19",
  "term_label": "eukaryotic translation initiation factor 3 complex"
}